autophagosome-dependent secretion [GO:0160192] (BP) References: PMID:25988755, PMID:38534758 Also known as: autophagy-dependent secretion, secretory autophagy Relationships: is a type of exocytosis [GO:0006887]; is a type of GO:0051656; is a type of autophagosome localization [GO:0061906] Definition: A process of exocytosis that uses the autophagy machinery to facilitate secretion of the cytosolic cargo such as leaderless cytosolic proteins which cannot enter the conventional secretory pathway operating via the endoplasmic reticulum and the Golgi apparatus.